positive regulation of ERK5 cascade [GO:0070378] (BP) Sources: GOC:mah Also known as: positive regulation of BMK cascade, positive regulation of BMK signaling pathway, positive regulation of BMK signalling pathway, positive regulation of BMK1 cascade, positive regulation of ERK5 signaling pathway, positive regulation of MAPK7 cascade, up regulation of BMK cascade, up-regulation of BMK cascade, upregulation of BMK cascade, activation of BMK cascade, stimulation of BMK cascade Definition: Any process that activates or increases the frequency, rate or extent of signal transduction mediated by the ERK5 cascade. Relationships: is a type of positive regulation of MAPK cascade [GO:0043410]; is a type of regulation of ERK5 cascade [GO:0070376]; RO_0002213 ERK5 cascade [GO:0070375]